{
  "gene_symbol": "CREG1",
  "gene_name": "Protein CREG1",
  "term_label": "Unknown biological process",
  "term_id": "UNKNOWN:0002",
  "gene": "UniProtKB:O75629"
}